{
  "gene_symbol": "NCAPH2",
  "gene_name": "Condensin-2 complex subunit H2",
  "term_label": "mitotic sister chromatid separation",
  "gene": "UniProtKB:Q6IBW4",
  "term_id": "GO:0051306"
}